{
  "gene": "UniProtKB:P28347",
  "term_label": "DNA-binding transcription factor activity, RNA polymerase II-specific",
  "term_id": "GO:0000981",
  "gene_symbol": "TEAD1",
  "gene_name": "Transcriptional enhancer factor TEF-1"
}